long-chain fatty acid import into peroxisome [GO:0015910] (biological process) Definition: The directed movement of a long-chain fatty acid into a peroxisome. A long-chain fatty acid has an aliphatic tail containing 13 to 22 carbons. Note: While there is not universal consensus on the lengths of short-, medium-, long- and very-long-chain fatty acids, the GO uses the definitions in ChEBI (see CHEBI:26666, CHEBI:59554, CHEBI:15904 and CHEBI:27283). Sources: GOC:ai Relationships: is a type of GO:0015909; is a type of peroxisomal membrane transport [GO:0015919]; is a type of GO:0032365; is a type of GO:1902001 Also known as: peroxisomal long-chain fatty acid import, peroxisomal long-chain fatty acid uptake